{
  "gene": "UniProtKB:Q5VYV0",
  "gene_name": "Forkhead box protein B2",
  "term_label": "anatomical structure morphogenesis",
  "term_id": "GO:0009653",
  "gene_symbol": "FOXB2"
}